{
  "term_id": "GO:0032266",
  "gene_symbol": "WIPI2",
  "gene_name": "WD repeat domain phosphoinositide-interacting protein 2",
  "term_label": "phosphatidylinositol-3-phosphate binding",
  "gene": "UniProtKB:Q9Y4P8"
}